bronchus development [GO:0060433] (biological process) Relationships: is a type of respiratory tube development [GO:0030323]; BFO_0000050 respiratory system development [GO:0060541] Subtypes: lobar bronchus development [GO:0060482] Definition: The biological process whose specific outcome is the progression of a bronchus from an initial condition to its mature state. This process begins with the formation of the bronchus and ends with the mature structure. The bronchus is the portion of the airway that connects to the lungs. Sources: GOC:dph